{
  "gene_symbol": "PLCL2",
  "term_id": "GO:0051209",
  "gene": "UniProtKB:Q9UPR0",
  "gene_name": "Inactive phospholipase C-like protein 2",
  "term_label": "release of sequestered calcium ion into cytosol"
}